dTDP-4-dehydro-6-deoxyglucose reductase activity [GO:0050573] (molecular function) Relationships: is a type of oxidoreductase activity, acting on the CH-OH group of donors, NAD or NADP as acceptor [GO:0016616] Sources: EC:1.1.1.266, RHEA:36583 Also known as: dTDP-4-keto-6-deoxyglucose reductase activity, dTDP-D-fucose:NADP+ oxidoreductase activity Definition: Catalysis of the reaction: dTDP-D-fucose + NADP+ = dTDP-4-dehydro-6-deoxy-alpha-D-glucose + H+ + NADPH.